{
  "term_id": "UNKNOWN:0003",
  "gene_name": "XK-related protein 3",
  "gene_symbol": "XKR3",
  "term_label": "Unknown cellular component",
  "gene": "UniProtKB:Q5GH77"
}